{
  "gene": "UniProtKB:Q9H2X9",
  "term_id": "GO:0055064",
  "gene_name": "Solute carrier family 12 member 5",
  "term_label": "chloride ion homeostasis",
  "gene_symbol": "SLC12A5"
}